T follicular helper cell differentiation [GO:0061470] (biological process) Definition: The process in which a relatively unspecialized T cell acquires specialized features of a mature T follicular helper cell. Also known as: T-helper follicular cell differentiation References: PMID:21572431 Sources: GOC:dph Relationships: is a type of T-helper cell differentiation [GO:0042093]